{
  "gene_symbol": "CFAP20DC",
  "gene": "UniProtKB:Q6ZVT6",
  "gene_name": "Protein CFAP20DC",
  "term_label": "Unknown cellular component",
  "term_id": "UNKNOWN:0003"
}